(25S)-Delta(7)-dafachronate binding [GO:1902052] (MF) References: PMID:16529801 Sources: GOC:TermGenie Definition: Binding to (25S)-Delta(7)-dafachronate. Relationships: is a type of carboxylic acid binding [GO:0031406]; is a type of steroid hormone binding [GO:1990239]